manoyl oxide synthase activity [GO:0062206] (molecular function) Relationships: is a type of carbon-oxygen lyase activity, acting on phosphates [GO:0016838] Definition: Catalysis of the reaction: 8-hydroxycopalyl diphosphate = (13R)-manoyl oxide + diphosphate. References: PMID:24990389 Sources: RHEA:54516